{
  "term_id": "GO:0004674",
  "gene_name": "Serine_threonine-protein kinase Nek6",
  "gene_symbol": "NEK6",
  "term_label": "protein serine/threonine kinase activity",
  "gene": "UniProtKB:Q9HC98"
}